lipid modification by small protein conjugation [GO:0120322] (biological process) Subtypes: lipid ubiquitination [GO:0120323] References: PMID:34012115 Sources: GOC:sp Definition: A lipid modification process in which one or more groups of a small protein, such as ubiquitin or a ubiquitin-like protein, are covalently attached to a target lipid. Relationships: is a type of lipid modification [GO:0030258]